symbiont-mediated suppression of host mRNA transcription via inhibition of RNA polymerase II activity [GO:0039523] (BP) Definition: A process in which a symbiont inhibits or disrupts the transcription of genes into mRNA in its host by directly inhibiting host RNA polymerase II activity. The host is defined as the larger of the organisms involved in a symbiotic interaction. References: PMID:25233083, PMID:36144426 Sources: GOC:bf, GOC:sp Relationships: is a type of GO:0039653 Also known as: inhibition of host RNA polymerase II by virus, inhibition of host RNA polymerase II activity by virus, negative regulation by virus of host RNA polymerase II activity, suppression by virus of host RNA polymerase II activity, suppression by virus of host mRNA transcription via inhibition of RNA polymerase II activity